{
  "gene_name": "Lipid transferase CIDEB",
  "term_id": "GO:0120013",
  "gene_symbol": "CIDEB",
  "gene": "UniProtKB:Q9UHD4",
  "term_label": "lipid transfer activity"
}